{
  "gene_symbol": "MMP9",
  "term_label": "extracellular matrix organization",
  "gene": "UniProtKB:P14780",
  "gene_name": "Matrix metalloproteinase-9",
  "term_id": "GO:0030198"
}